{
  "term_label": "Unknown molecular function",
  "gene_name": "Zinc finger BED domain-containing protein 6",
  "term_id": "UNKNOWN:0001",
  "gene_symbol": "ZBED6",
  "gene": "UniProtKB:P86452"
}